amino acid ligation activity by nonribosomal peptide synthase [GO:0097429] (molecular function) Definition: Catalysis of the ligation of an amino acid to another amino acid via a carbon-nitrogen bond, with the concomitant hydrolysis of the diphosphate bond in ATP or a similar triphosphate, carried out by a nonribosomal peptide synthase. Relationships: is a type of acid-amino acid ligase activity [GO:0016881]; is a type of GO:1904091 Sources: GOC:vw